substituted mannan metabolic process [GO:0006080] (biological process) Relationships: is a type of polysaccharide metabolic process [GO:0005976] Subtypes: GO:0010391, galactoglucomannan metabolic process [GO:0010392], galactomannan metabolic process [GO:0051069] Also known as: substituted mannan metabolism Sources: GOC:tair_curators Definition: The chemical reactions and pathways involving a mannan backbone composed of D-mannose unites, substituted with D-glucose and/or D-galactose units.